{
  "term_label": "interleukin-15-mediated signaling pathway",
  "gene_name": "T-cell surface glycoprotein CD4",
  "gene": "UniProtKB:P01730",
  "gene_symbol": "CD4",
  "term_id": "GO:0035723"
}